replication fork processing [GO:0031297] (biological process) Relationships: is a type of DNA-templated DNA replication maintenance of fidelity [GO:0045005] Also known as: collapsed replication fork processing, recovery from replication fork arrest, recovery from replication fork stalling, recovery from replication fork arrest at rDNA locus, recovery from replication fork stalling at rDNA locus, replication fork processing at rDNA locus, replication fork processing at ribosomal DNA locus, replication fork restart, replication restart Definition: The process in which a DNA replication fork that has stalled is restored to a functional state and replication is restarted. The stalling may be due to DNA damage, DNA secondary structure, bound proteins, dNTP shortage, or other causes. References: PMID:11459955, PMID:15367656, PMID:17660542 Sources: GOC:vw Subtypes: replication fork reversal [GO:0071932], mitotic recombination-dependent replication fork processing [GO:1990426]